{
  "gene_symbol": "KHDRBS3",
  "gene_name": "KH domain-containing, RNA-binding, signal transduction-associated protein 3",
  "term_label": "regulation of alternative mRNA splicing, via spliceosome",
  "term_id": "GO:0000381",
  "gene": "UniProtKB:O75525"
}